{
  "term_label": "negative regulation of TORC1 signaling",
  "gene_symbol": "NPRL3",
  "term_id": "GO:1904262",
  "gene": "UniProtKB:Q12980",
  "gene_name": "GATOR complex protein NPRL3"
}